negative regulation of neutrophil activation [GO:1902564] (biological process) References: PMID:17588661 Sources: GOC:TermGenie Relationships: is_a negative regulation of leukocyte activation [GO:0002695]; is a type of regulation of neutrophil activation [GO:1902563]; negatively regulates neutrophil activation [GO:0042119] Also known as: down regulation of neutrophil activation, down-regulation of neutrophil activation, downregulation of neutrophil activation, inhibition of neutrophil activation Definition: Any process that stops, prevents or reduces the frequency, rate or extent of neutrophil activation.